mesenchymal stem cell maintenance involved in metanephric nephron morphogenesis [GO:0072309] (biological process) Relationships: is a type of GO:0072038; is part of metanephric nephron morphogenesis [GO:0072273] Regulation: regulated by regulation of mesenchymal cell apoptotic process involved in metanephric nephron morphogenesis [GO:0072304]; negatively regulated by negative regulation of mesenchymal cell apoptotic process involved in metanephric nephron morphogenesis [GO:0072305]; positively regulated by positive regulation of mesenchymal cell apoptotic process involved in metanephric nephron morphogenesis [GO:0072306] Definition: The process in which an organism retains a population of mesenchymal stem cells that contributes to the shaping of a nephron in the metanephros. A mesenchymal stem cell is a cell that retains the ability to divide and proliferate throughout life to provide progenitor cells that can differentiate into specialized mesenchymal cells. Sources: GOC:mtg_kidney_jan10